{
  "gene_name": "Protein FAM72C",
  "gene_symbol": "FAM72C",
  "term_label": "Unknown molecular function",
  "gene": "UniProtKB:H0Y354",
  "term_id": "UNKNOWN:0001"
}